{
  "gene_symbol": "MAD2L1",
  "term_id": "UNKNOWN:0001",
  "gene": "UniProtKB:Q13257",
  "gene_name": "Mitotic spindle assembly checkpoint protein MAD2A",
  "term_label": "Unknown molecular function"
}